vestibular receptor cell development [GO:0060118] (biological process) Definition: The process whose specific outcome is the progression of a vestibular receptor cell over time, from its formation to the mature structure. Cell development does not include the steps involved in committing a cell to a specific fate. Relationships: is a type of inner ear receptor cell development [GO:0060119]; is part of GO:0060114 Also known as: vestibular hair cell development Sources: GOC:dph